HNK-1 sulfotransferase activity [GO:0016232] (MF) Definition: Catalysis of the synthesis of the HKK-1 carbohydrate epitope; adds a sulfate group to a precursor, GlcA-beta-(1->3)-Gal-beta-(1->4)-GlcNAc-beta-(1->R), forming sulfo-3GlcA-beta-(1->3)-Gal-beta-(1->4)-GlcNAc-beta-(1->R). Relationships: is a type of sulfotransferase activity [GO:0008146] References: PMID:9478973 Also known as: HNK-1 sulphotransferase activity